response to dietary excess [GO:0002021] (biological process) Definition: The physiological process in which dietary excess is sensed by the central nervous system, resulting in a reduction in food intake and increased energy expenditure. References: PMID:12161655 Sources: GOC:pg, GOC:pr Relationships: is a type of response to nutrient levels [GO:0031667]; is a type of energy homeostasis [GO:0097009]